pyruvate fermentation to propionate [GO:0019657] (biological process) Also known as: succinate-propionate fermentation, glycolytic fermentation to propionate Definition: The anaerobic chemical reactions and pathways resulting in the breakdown of pyruvate into to propionate, an alternative to the acrylate pathway to produce propionate. Sources: GOC:dph, GOC:nr, MetaCyc:P108-PWY Relationships: is a type of succinate metabolic process [GO:0006105]; is a type of GO:0019541; is a type of pyruvate fermentation [GO:0019660]; has part propionyl-CoA:succinate CoA-transferase activity [GO:0043821]; has part methylmalonyl-CoA carboxytransferase activity [GO:0047154]